{
  "gene": "UniProtKB:Q8WVF2",
  "term_label": "embryonic skeletal system development",
  "term_id": "GO:0048706",
  "gene_name": "Unique cartilage matrix-associated protein",
  "gene_symbol": "UCMA"
}